guanosine kinase activity [GO:0106366] (molecular function) References: PMID:10879466, PMID:7665468 Sources: RHEA:27710 Definition: Catalysis of the reaction: ATP + guanosine = ADP + GMP. Relationships: is a type of nucleoside kinase activity [GO:0019206]